{
  "term_id": "GO:0004222",
  "gene": "UniProtKB:Q9P2N4",
  "term_label": "metalloendopeptidase activity",
  "gene_name": "A disintegrin and metalloproteinase with thrombospondin motifs 9",
  "gene_symbol": "ADAMTS9"
}